{
  "term_id": "GO:0006508",
  "term_label": "proteolysis",
  "gene_name": "A disintegrin and metalloproteinase with thrombospondin motifs 18",
  "gene_symbol": "ADAMTS18",
  "gene": "UniProtKB:Q8TE60"
}